{
  "term_label": "Unknown biological process",
  "term_id": "UNKNOWN:0002",
  "gene_name": "Headcase protein homolog",
  "gene_symbol": "HECA",
  "gene": "UniProtKB:Q9UBI9"
}